{
  "gene_name": "NudC domain-containing protein 2",
  "term_label": "cytoplasm",
  "gene_symbol": "NUDCD2",
  "term_id": "GO:0005737",
  "gene": "UniProtKB:Q8WVJ2"
}